imaginal disc-derived leg morphogenesis [GO:0007480] (biological process) Definition: The process in which the anatomical structures of a leg derived from an imaginal disc are generated and organized. A leg is a limb on which an animal walks and stands. An example of this is found in Drosophila melanogaster. Relationships: is a type of imaginal disc-derived appendage morphogenesis [GO:0035114]; is a type of post-embryonic appendage morphogenesis [GO:0035120]; is part of GO:0007478 Sources: GOC:mtg_sensu, ISBN:0879694238 Regulation: regulated by GO:0110137; positively regulated by positive regulation of imaginal disc-derived leg joint morphogenesis [GO:0110138]; negatively regulated by negative regulation of imaginal disc-derived leg joint morphogenesis [GO:0110139]